{
  "gene_name": "Protein FAM53C",
  "term_id": "UNKNOWN:0001",
  "gene_symbol": "FAM53C",
  "term_label": "Unknown molecular function",
  "gene": "UniProtKB:Q9NYF3"
}